{
  "term_label": "chloride channel activity",
  "gene_name": "Chloride intracellular channel protein 1",
  "gene_symbol": "CLIC1",
  "term_id": "GO:0005254",
  "gene": "UniProtKB:O00299"
}